TRIBOA-glucoside methyltransferase activity [GO:0102718] (molecular function) Relationships: is a type of methyltransferase activity [GO:0008168] Sources: EC:2.1.1.241, GOC:pz Definition: Catalysis of the reaction: TRIBOA-beta-D-glucoside + S-adenosyl-L-methionine = (2R)-DIMBOA glucoside + S-adenosyl-L-homocysteine + H+.